{
  "gene_name": "Gametocyte-specific factor 1",
  "term_id": "UNKNOWN:0002",
  "gene_symbol": "GTSF1",
  "term_label": "Unknown biological process",
  "gene": "UniProtKB:Q8WW33"
}